{
  "term_id": "GO:0008429",
  "gene_name": "Extended synaptotagmin-3",
  "gene_symbol": "ESYT3",
  "gene": "UniProtKB:A0FGR9",
  "term_label": "phosphatidylethanolamine binding"
}